{
  "term_id": "GO:0060349",
  "term_label": "bone morphogenesis",
  "gene_name": "Interferon-induced transmembrane protein 5",
  "gene": "UniProtKB:A6NNB3",
  "gene_symbol": "IFITM5"
}